{
  "term_id": "GO:0015485",
  "gene": "UniProtKB:P35610",
  "term_label": "cholesterol binding",
  "gene_symbol": "SOAT1",
  "gene_name": "Sterol O-acyltransferase 1"
}